regulation of interleukin-5 production [GO:0032674] (biological process) Also known as: regulation of IL-5 production, regulation of interleukin-5 biosynthetic process, regulation of interleukin-5 secretion Subtypes: negative regulation of interleukin-5 production [GO:0032714], positive regulation of interleukin-5 production [GO:0032754] Sources: GOC:mah Relationships: is a type of regulation of cytokine production [GO:0001817]; regulates interleukin-5 production [GO:0032634] Definition: Any process that modulates the frequency, rate, or extent of interleukin-5 production.